DNA recombination [GO:0006310] (biological process) Regulation: regulated by GO:0000018; negatively regulated by negative regulation of DNA recombination [GO:0045910]; RO_0002213 by positive regulation of DNA recombination [GO:0045911] Subtypes: recombinational repair [GO:0000725], mitotic recombination [GO:0006312], DNA transposition [GO:0006313], GO:0006314, GO:0016444, homologous recombination [GO:0035825], plasmid recombination [GO:0042150], RNA-mediated DNA recombination [GO:0042152], recombination within rDNA repeats [GO:0045458], mitochondrion DNA recombination [GO:1905951], intrachromosomal DNA recombination [GO:1990067] Relationships: is a type of DNA metabolic process [GO:0006259] Sources: ISBN:0198506732 Definition: Any process in which a new genotype is formed by reassortment of genes resulting in gene combinations different from those that were present in the parents. In eukaryotes genetic recombination can occur by chromosome assortment, intrachromosomal recombination, or nonreciprocal interchromosomal recombination. Interchromosomal recombination occurs by crossing over. In bacteria it may occur by genetic transformation, conjugation, transduction, or F-duction.